interleukin-31 production [GO:0072635] (biological process) Relationships: is a type of cytokine production [GO:0001816] References: PMID:30328794 Sources: GOC:BHF, GOC:mah Also known as: IL-31 production, interleukin-31 secretion Definition: The appearance of interleukin-31 due to biosynthesis or secretion following a cellular stimulus, resulting in an increase in its intracellular or extracellular levels.